{
  "gene": "UniProtKB:Q9Y231",
  "gene_name": "4-galactosyl-N-acetylglucosaminide 3-alpha-L-fucosyltransferase 9",
  "term_label": "4-galactosyl-N-acetylglucosaminide 3-alpha-L-fucosyltransferase activity",
  "gene_symbol": "FUT9",
  "term_id": "GO:0017083"
}